{
  "gene": "UniProtKB:P19544",
  "gene_symbol": "WT1",
  "gene_name": "Wilms tumor protein",
  "term_id": "GO:0000978",
  "term_label": "RNA polymerase II cis-regulatory region sequence-specific DNA binding"
}